{
  "gene_name": "Transcription factor E4F1",
  "gene_symbol": "E4F1",
  "term_id": "GO:0006357",
  "gene": "UniProtKB:Q66K89",
  "term_label": "regulation of transcription by RNA polymerase II"
}